{
  "gene_symbol": "CPA6",
  "term_id": "GO:0005615",
  "gene_name": "Carboxypeptidase A6",
  "gene": "UniProtKB:Q8N4T0",
  "term_label": "extracellular space"
}